{
  "gene": "UniProtKB:P07476",
  "term_id": "GO:0060090",
  "term_label": "molecular adaptor activity",
  "gene_symbol": "IVL",
  "gene_name": "Involucrin"
}